{
  "term_label": "Unknown molecular function",
  "term_id": "UNKNOWN:0001",
  "gene_symbol": "TRAV8-3",
  "gene_name": "T cell receptor alpha variable 8-3",
  "gene": "UniProtKB:A0A0A6YYJ7"
}